{
  "gene_name": "Methionine--tRNA ligase, cytoplasmic",
  "gene_symbol": "MARS1",
  "term_label": "methionyl-tRNA aminoacylation",
  "term_id": "GO:0006431",
  "gene": "UniProtKB:P56192"
}